{
  "gene": "UniProtKB:P68363",
  "gene_symbol": "TUBA1B",
  "gene_name": "Tubulin alpha-1B chain",
  "term_id": "GO:0005874",
  "term_label": "microtubule"
}